{
  "gene": "UniProtKB:Q86VS3",
  "gene_symbol": "IQCH",
  "term_id": "UNKNOWN:0003",
  "gene_name": "IQ domain-containing protein H",
  "term_label": "Unknown cellular component"
}